{
  "term_id": "UNKNOWN:0001",
  "gene": "UniProtKB:Q99440",
  "term_label": "Unknown molecular function",
  "gene_name": "Uncharacterized protein encoded by LINC01587",
  "gene_symbol": "LINC01587"
}